{
  "term_label": "cytokine activity",
  "term_id": "GO:0005125",
  "gene_symbol": "WNT2",
  "gene": "UniProtKB:P09544",
  "gene_name": "Protein Wnt-2"
}